{
  "gene_symbol": "PRSS36",
  "term_label": "Unknown cellular component",
  "gene": "UniProtKB:Q5K4E3",
  "gene_name": "Polyserase-2",
  "term_id": "UNKNOWN:0003"
}